{
  "gene_name": "MICOS complex subunit MIC13",
  "gene": "UniProtKB:Q5XKP0",
  "term_id": "GO:0044284",
  "term_label": "mitochondrial crista junction",
  "gene_symbol": "MICOS13"
}